{
  "gene_name": "Kinocilin",
  "term_id": "GO:0016324",
  "gene": "UniProtKB:A6PVL3",
  "term_label": "apical plasma membrane",
  "gene_symbol": "KNCN"
}